negative regulation of BMP secretion [GO:2001285] (biological process) Also known as: negative regulation of BMP protein secretion, negative regulation of bone morphogenetic protein secretion Definition: Any process that stops, prevents or reduces the frequency, rate or extent of BMP secretion. Relationships: is a type of negative regulation of cell communication [GO:0010648]; is a type of negative regulation of signaling [GO:0023057]; is a type of GO:0050709; is a type of GO:2001284; negatively regulates BMP secretion [GO:0038055] Sources: GOC:sart